{
  "gene_name": "Zinc finger protein 10",
  "gene_symbol": "ZNF10",
  "gene": "UniProtKB:P21506",
  "term_label": "DNA-binding transcription factor activity, RNA polymerase II-specific",
  "term_id": "GO:0000981"
}